{
  "gene_symbol": "A0A669KAW2",
  "term_label": "Unknown cellular component",
  "gene": "UniProtKB:A0A669KAW2",
  "term_id": "UNKNOWN:0003",
  "gene_name": "Uncharacterized protein"
}